mitochondrial double-strand break repair [GO:0097551] (biological process) Also known as: mtDSB repair Note: Note that the processes of nuclear double-strand break repair and mitochondrial double-strand break repair are genetically separable. References: PMID:22214610 Sources: GOC:di Relationships: is a type of double-strand break repair [GO:0006302] Definition: The repair of double-strand breaks in mitochondrial DNA via homologous and nonhomologous mechanisms to reform a continuous DNA helix. Subtypes: mitochondrial double-strand break repair via homologous recombination [GO:0097552]